{
  "gene_symbol": "SLC20A2",
  "gene": "UniProtKB:Q08357",
  "term_label": "phosphate ion transmembrane transport",
  "term_id": "GO:0035435",
  "gene_name": "Sodium-dependent phosphate transporter 2"
}